CXCL12-activated CXCR4 signaling pathway [GO:0038160] (biological process) Also known as: CXCL12-activated CXCR4 signalling pathway Sources: GOC:nhn Definition: The series of molecular signals initiated by the binding of the C-X-C chemokine CXCL12 to a C-X-C chemokine type 4 receptor (CXCR4) on the surface of a target cell, and ending with the regulation of a downstream cellular process, e.g. transcription. Relationships: is a type of chemokine (C-X-C motif) ligand 12 signaling pathway [GO:0038146]; is a type of C-X-C chemokine receptor CXCR4 signaling pathway [GO:0038159]